{
  "term_label": "regulation of transcription by RNA polymerase II",
  "term_id": "GO:0006357",
  "gene_name": "Sal-like protein 3",
  "gene_symbol": "SALL3",
  "gene": "UniProtKB:Q9BXA9"
}